{
  "term_id": "GO:0005794",
  "term_label": "Golgi apparatus",
  "gene": "UniProtKB:Q49A17",
  "gene_symbol": "GALNTL6",
  "gene_name": "Polypeptide N-acetylgalactosaminyltransferase-like 6"
}